{
  "gene_name": "SUMO-conjugating enzyme UBC9",
  "gene_symbol": "UBE2I",
  "term_label": "protein sumoylation",
  "term_id": "GO:0016925",
  "gene": "UniProtKB:P63279"
}